{
  "gene_symbol": "TRAJ18",
  "term_id": "UNKNOWN:0002",
  "term_label": "Unknown biological process",
  "gene_name": "T cell receptor alpha joining 18 (Fragment)",
  "gene": "UniProtKB:A0A075B6X9"
}